{
  "term_id": "GO:0005834",
  "gene_name": "Guanine nucleotide-binding protein G(t) subunit alpha-3",
  "gene": "UniProtKB:A8MTJ3",
  "gene_symbol": "GNAT3",
  "term_label": "heterotrimeric G-protein complex"
}